{
  "gene_symbol": "ZFAT",
  "gene": "UniProtKB:Q9P243",
  "term_id": "UNKNOWN:0003",
  "term_label": "Unknown cellular component",
  "gene_name": "Zinc finger protein ZFAT"
}